sucrose catabolic process via 3'-ketosucrose [GO:0019574] (biological process) Relationships: is a type of sucrose catabolic process [GO:0005987]; is a type of glucose metabolic process [GO:0006006]; is a type of GO:0006796; is a type of organophosphate metabolic process [GO:0019637]; is a type of GO:1901135; has part fructokinase activity [GO:0008865]; has part GO:0033757; has part 3-ketoglucose-reductase activity [GO:0048258] Definition: The chemical reactions and pathways resulting in the breakdown of sucrose, which proceeds via the conversion of sucrose to 3'-ketosucrose. 3'-ketosucrose is hydrolyzed to 3-ketoglucose and fructose, and the 3-ketoglucose is then be converted to glucose. Also known as: sucrose breakdown, using glucoside 3-dehydrogenase, sucrose catabolic process to D-glucose, sucrose catabolic process, using glucoside 3-dehydrogenase, sucrose catabolism, using glucoside 3-dehydrogenase, sucrose degradation, using glucoside 3-dehydrogenase Sources: GOC:bf, GOC:dgf, MetaCyc:SUCROSEUTIL2-PWY